{
  "term_label": "Unknown biological process",
  "gene": "UniProtKB:O14737",
  "gene_name": "Programmed cell death protein 5",
  "gene_symbol": "PDCD5",
  "term_id": "UNKNOWN:0002"
}